{
  "term_label": "ubiquitin protein ligase binding",
  "gene_symbol": "GABARAPL1",
  "gene_name": "Gamma-aminobutyric acid receptor-associated protein-like 1",
  "term_id": "GO:0031625",
  "gene": "UniProtKB:Q9H0R8"
}